{
  "gene": "UniProtKB:Q13613",
  "term_id": "GO:0052629",
  "term_label": "phosphatidylinositol-3,5-bisphosphate 3-phosphatase activity",
  "gene_name": "Myotubularin-related protein 1",
  "gene_symbol": "MTMR1"
}